{
  "gene_name": "Trafficking protein particle complex subunit 12",
  "term_label": "Golgi apparatus",
  "term_id": "GO:0005794",
  "gene_symbol": "TRAPPC12",
  "gene": "UniProtKB:Q8WVT3"
}